{
  "gene_symbol": "TAFAZZIN",
  "gene_name": "Tafazzin",
  "term_label": "1-acylglycerophosphocholine O-acyltransferase activity",
  "term_id": "GO:0047184",
  "gene": "UniProtKB:Q16635"
}